alpha-1,4-glucan glucosyltransferase (ADP-glucose donor) activity [GO:0009011] (molecular function) Definition: Catalysis of the reaction: [(1->4)-alpha-D-glucosyl](n) + ADP-alpha-D-glucose = [(1->4)-alpha-D-glucosyl](n+1) + ADP + H+. Also known as: ADP-glucose transglucosylase activity, ADP-glucose:1,4-alpha-D-glucan 4-alpha-D-glucosyltransferase activity, ADPG starch synthetase activity, ADPG-starch glucosyltransferase activity, ADPglucose-starch glucosyltransferase activity, ADPglucose:1,4-alpha-D-glucan 4-alpha-D-glucosyltransferase activity, adenosine diphosphate glucose-starch glucosyltransferase activity, adenosine diphosphoglucose-starch glucosyltransferase activity, starch synthase activity, starch synthetase activity, starch (bacterial glycogen) synthase activity, ADP-glucose starch synthase activity, ADP-glucose--starch glucosyltransferase activity, glycogen synthase activity Sources: RHEA:18189 Relationships: is a type of alpha-1,4-glucan glucosyltransferase (NDP-glucose donor) activity [GO:0033840]